{
  "gene_symbol": "SLC22A1",
  "gene": "UniProtKB:O15245",
  "gene_name": "Solute carrier family 22 member 1",
  "term_id": "GO:0015695",
  "term_label": "organic cation transport"
}